{
  "gene": "UniProtKB:Q86UF2",
  "term_id": "GO:0005789",
  "gene_name": "cTAGE family member 6",
  "gene_symbol": "CTAGE6",
  "term_label": "endoplasmic reticulum membrane"
}